{
  "gene": "UniProtKB:Q9NR20",
  "term_id": "GO:0005737",
  "gene_name": "Dual specificity tyrosine-phosphorylation-regulated kinase 4",
  "gene_symbol": "DYRK4",
  "term_label": "cytoplasm"
}